antigen processing and presentation of endogenous peptide antigen via MHC class Ib via ER pathway [GO:0002488] (biological process) Definition: The process in which an antigen-presenting cell expresses a peptide antigen of endogenous origin on its cell surface in association with an MHC class Ib protein complex following intracellular transport via an ER pathway. The peptide is typically a fragment of a larger endogenous protein which has been degraded within the cell and becomes associated with the MHC class Ib molecule in the ER. Class Ib here refers to non-classical class I molecules, such as those of the HLA-E gene family. References: PMID:15928678 Sources: GOC:add Relationships: is a type of antigen processing and presentation of endogenous peptide antigen via MHC class Ib [GO:0002476] Subtypes: antigen processing and presentation of endogenous peptide antigen via MHC class Ib via ER pathway, TAP-dependent [GO:0002489], antigen processing and presentation of endogenous peptide antigen via MHC class Ib via ER pathway, TAP-independent [GO:0002490] Also known as: endogenous peptide antigen processing and presentation via MHC class Ib via ER pathway